{
  "gene": "UniProtKB:Q8N7H5",
  "term_id": "UNKNOWN:0002",
  "term_label": "Unknown biological process",
  "gene_name": "RNA polymerase II-associated factor 1 homolog",
  "gene_symbol": "PAF1"
}